{
  "gene": "UniProtKB:O75290",
  "term_id": "GO:0000978",
  "gene_name": "Zinc finger protein 780A",
  "gene_symbol": "ZNF780A",
  "term_label": "RNA polymerase II cis-regulatory region sequence-specific DNA binding"
}